regulation of somitomeric trunk muscle development [GO:0014708] (BP) Definition: Any process that modulates the frequency, rate or extent of somitomeric trunk muscle development. Sources: GOC:mtg_muscle Subtypes: positive regulation of somitomeric trunk muscle development [GO:0014709], negative regulation of somitomeric trunk muscle development [GO:0014710] Relationships: is a type of regulation of muscle organ development [GO:0048634]; regulates GO:0002075